{
  "term_id": "GO:0003073",
  "gene_symbol": "KLK2",
  "gene": "UniProtKB:P20151",
  "gene_name": "Kallikrein-2",
  "term_label": "regulation of systemic arterial blood pressure"
}